lipopolysaccharide biosynthetic process [GO:0009103] (biological process) Definition: The chemical reactions and pathways resulting in the formation of lipopolysaccharides, any of a group of related, structurally complex components of the outer membrane of Gram-negative bacteria. Sources: GOC:ai, GOC:mr Also known as: LPS biosynthetic process, lipopolysaccharide anabolism, lipopolysaccharide biosynthesis, lipopolysaccharide formation, lipopolysaccharide synthesis Relationships: is a type of GO:0000271; is a type of lipid biosynthetic process [GO:0008610]; is a type of GO:0008653; is_a carbohydrate derivative biosynthetic process [GO:1901137]